{
  "gene_symbol": "IGFL1",
  "gene": "UniProtKB:Q6UW32",
  "term_label": "Unknown biological process",
  "gene_name": "Insulin growth factor-like family member 1",
  "term_id": "UNKNOWN:0002"
}